{
  "term_label": "positive regulation of cAMP/PKA signal transduction",
  "gene": "UniProtKB:P01286",
  "gene_name": "Somatoliberin",
  "term_id": "GO:0141163",
  "gene_symbol": "GHRH"
}